{
  "gene": "UniProtKB:Q8IUR5",
  "gene_name": "Protein O-mannosyl-transferase TMTC1",
  "term_label": "mannosyltransferase activity",
  "term_id": "GO:0000030",
  "gene_symbol": "TMTC1"
}